{
  "term_id": "GO:0005886",
  "term_label": "plasma membrane",
  "gene": "UniProtKB:Q92482",
  "gene_name": "Aquaporin-3",
  "gene_symbol": "AQP3"
}